nodal signaling pathway [GO:0038092] (biological process) Definition: The series of molecular signals initiated by nodal protein binding to an activin receptor on the surface of a target cell, and ending with the regulation of a downstream cellular process, e.g. transcription. References: PMID:17287255 Sources: GOC:BHF, GOC:vk Also known as: nodal signaling, nodal signalling pathway Relationships: is a type of activin receptor signaling pathway [GO:0032924] Regulation: positively regulated by GO:0141092; regulated by regulation of nodal signaling pathway [GO:1900107]; negatively regulated by negative regulation of nodal signaling pathway [GO:1900108]